{
  "gene": "UniProtKB:P30084",
  "term_label": "mitochondrion",
  "gene_name": "Enoyl-CoA hydratase, mitochondrial",
  "term_id": "GO:0005739",
  "gene_symbol": "ECHS1"
}